regulation of pectin catabolic process [GO:2001003] (BP) Definition: Any process that modulates the frequency, rate or extent of pectin catabolic process. Also known as: regulation of pectin breakdown, regulation of pectin catabolism, regulation of pectin degradation Relationships: is a type of GO:0032881; is a type of regulation of carbohydrate catabolic process [GO:0043470]; regulates pectin catabolic process [GO:0045490] Subtypes: negative regulation of pectin catabolic process [GO:2001004], positive regulation of pectin catabolic process [GO:2001005] Sources: GOC:mengo_curators